{
  "term_id": "UNKNOWN:0001",
  "gene": "UniProtKB:Q6ZSJ8",
  "gene_name": "Uncharacterized protein C1orf122",
  "term_label": "Unknown molecular function",
  "gene_symbol": "C1orf122"
}